macropinosome membrane [GO:0160056] (cellular component) References: PMID:19690049 Definition: The lipid bilayer surrounding a macropinosome. Relationships: is a type of endosome membrane [GO:0010008]; is part of macropinosome [GO:0044354]